histone H4K91 ubiquitin ligase activity [GO:0141000] (MF) Relationships: is a type of histone H4 ubiquitin ligase activity [GO:0141056] References: PMID:19818714 Definition: Catalysis of the transfer of a ubiquitin molecule to histone 4 at the lysine-91 residue. Note: Note that the residue position corresponds to the canonical human H4 histone (UniProtKB:P02309); this residue is conserved across all eukaryotes. Note that the initiation methionine is cleaved, so the first residue is S1. Also known as: histone H4-K91 ubiquitin ligase activity, histone ubiquitin ligase activity (H4-K91 specific)